protein localization to cytosolic proteasome complex [GO:1904327] (BP) Also known as: protein localisation in cytosolic proteasome complex, protein localisation to cytosolic proteasome complex, protein localization in cytosolic proteasome complex Definition: A process in which a protein is transported to, or maintained in, a location within a cytosolic proteasome complex. Relationships: is a type of intracellular protein localization [GO:0008104] References: PMID:17000876 Sources: GOC:PARL, GOC:TermGenie, GOC:bf, GO_REF:0000087